{
  "gene_name": "Polyubiquitin-C",
  "gene": "UniProtKB:P0CG48",
  "term_id": "GO:0031386",
  "gene_symbol": "UBC",
  "term_label": "protein tag activity"
}